{
  "gene_name": "Huntingtin-associated protein 1",
  "gene": "UniProtKB:P54257",
  "gene_symbol": "HAP1",
  "term_id": "GO:0048011",
  "term_label": "neurotrophin TRK receptor signaling pathway"
}